{
  "term_id": "GO:0005739",
  "gene": "UniProtKB:Q9UII2",
  "gene_name": "ATPase inhibitor, mitochondrial",
  "gene_symbol": "ATP5IF1",
  "term_label": "mitochondrion"
}